has_scope [oboInOwl#hasScope]